sulfur reductase activity [GO:0033796] (molecular function) Also known as: sulphur reductase activity, (donor):sulfur oxidoreductase activity Relationships: is a type of GO:0046995 Sources: RHEA:35591 Definition: Catalysis of the reduction of elemental sulfur or polysulfide to hydrogen sulfide, H2 + n sulfur = H+ + hydrogen sulfide + (n-1) sulfur.